{
  "gene_name": "DPY30 domain-containing protein 1",
  "gene": "UniProtKB:Q8WWB3",
  "term_id": "UNKNOWN:0002",
  "term_label": "Unknown biological process",
  "gene_symbol": "DYDC1"
}